{
  "gene_symbol": "DTWD1",
  "gene_name": "tRNA-uridine aminocarboxypropyltransferase 1",
  "term_label": "tRNA modification",
  "term_id": "GO:0006400",
  "gene": "UniProtKB:Q8N5C7"
}